{
  "term_id": "GO:1990112",
  "gene": "UniProtKB:O94822",
  "gene_symbol": "LTN1",
  "gene_name": "E3 ubiquitin-protein ligase listerin",
  "term_label": "RQC complex"
}